{
  "gene_name": "Max dimerization protein 4",
  "term_id": "GO:0000981",
  "term_label": "DNA-binding transcription factor activity, RNA polymerase II-specific",
  "gene_symbol": "MXD4",
  "gene": "UniProtKB:Q14582"
}